{
  "gene_symbol": "CLPTM1",
  "term_label": "membrane",
  "term_id": "GO:0016020",
  "gene": "UniProtKB:O96005",
  "gene_name": "Putative lipid scramblase CLPTM1"
}